{
  "gene": "UniProtKB:P49759",
  "gene_symbol": "CLK1",
  "term_label": "nucleus",
  "gene_name": "Dual specificity protein kinase CLK1",
  "term_id": "GO:0005634"
}